{
  "gene": "UniProtKB:P02545",
  "term_label": "heterochromatin formation",
  "gene_name": "Prelamin-A_C",
  "gene_symbol": "LMNA",
  "term_id": "GO:0031507"
}